{
  "term_label": "endosome",
  "term_id": "GO:0005768",
  "gene_name": "TOM1-like protein 2",
  "gene": "UniProtKB:Q6ZVM7",
  "gene_symbol": "TOM1L2"
}